{
  "gene_symbol": "TXNDC8",
  "gene": "UniProtKB:Q6A555",
  "gene_name": "Thioredoxin domain-containing protein 8",
  "term_label": "spermatogenesis",
  "term_id": "GO:0007283"
}